{
  "gene_name": "DNA dC-dU-editing enzyme APOBEC-3A",
  "gene": "UniProtKB:P31941",
  "term_label": "nucleus",
  "gene_symbol": "APOBEC3A",
  "term_id": "GO:0005634"
}